{
  "term_label": "extracellular matrix",
  "gene_name": "Collagen alpha-5(VI) chain",
  "term_id": "GO:0031012",
  "gene_symbol": "COL6A5",
  "gene": "UniProtKB:A8TX70"
}